protein localization to cell periphery [GO:1990778] (biological process) References: PMID:18216290 Regulation: regulated by regulation of protein localization to cell periphery [GO:1904375]; negatively regulated by GO:1904376; positively regulated by positive regulation of protein localization to cell periphery [GO:1904377] Definition: A process in which a protein is transported to, or maintained in, the cell periphery. Subtypes: GO:0044860, protein transport out of plasma membrane raft [GO:0044862], GO:0072659, GO:0072697, GO:0089705, GO:0098877, GO:0099613, protein localization to spore cell wall [GO:0099614], protein localization to presynaptic membrane [GO:0099644], endocytosis, site selection [GO:0120207], protein localization to basolateral plasma membrane [GO:1903361], protein localization to plasma membrane of cell tip [GO:1903418], protein localization to ciliary membrane [GO:1903441], protein localization to postsynaptic membrane [GO:1903539], protein localization to microvillus membrane [GO:1904107], GO:1905345 Relationships: is a type of intracellular protein localization [GO:0008104]